positive regulation of cytosolic calcium ion concentration involved in egg activation [GO:0060470] (biological process) Also known as: elevation of cytosolic calcium ion concentration involved in egg activation Relationships: is a type of positive regulation of cytosolic calcium ion concentration [GO:0007204]; is part of egg activation [GO:0007343] Definition: The process that increases the concentration of calcium ions in the cytosol after fertilization or the physiological activation of an egg. Sources: GOC:dph Subtypes: positive regulation of cortical granule exocytosis by positive regulation of cytosolic calcium ion concentration [GO:0060472]